{
  "gene_name": "Syntaxin-18",
  "gene_symbol": "STX18",
  "term_id": "GO:0005783",
  "term_label": "endoplasmic reticulum",
  "gene": "UniProtKB:Q9P2W9"
}